{
  "gene": "UniProtKB:P35251",
  "gene_name": "Replication factor C subunit 1",
  "term_label": "DNA binding",
  "gene_symbol": "RFC1",
  "term_id": "GO:0003677"
}